{
  "term_id": "GO:0070936",
  "term_label": "protein K48-linked ubiquitination",
  "gene_name": "Ubiquitin-conjugating enzyme E2 D3",
  "gene": "UniProtKB:P61077",
  "gene_symbol": "UBE2D3"
}